{
  "gene_name": "Keratin-associated protein 1-3",
  "term_label": "Unknown molecular function",
  "gene": "UniProtKB:Q8IUG1",
  "gene_symbol": "KRTAP1-3",
  "term_id": "UNKNOWN:0001"
}